{
  "term_id": "GO:0004984",
  "gene_symbol": "OR51A4",
  "gene_name": "Olfactory receptor 51A4",
  "gene": "UniProtKB:Q8NGJ6",
  "term_label": "olfactory receptor activity"
}